{
  "gene": "UniProtKB:Q9NX61",
  "gene_name": "Transmembrane protein 161A",
  "gene_symbol": "TMEM161A",
  "term_id": "UNKNOWN:0001",
  "term_label": "Unknown molecular function"
}